{
  "gene": "UniProtKB:P62324",
  "term_label": "cytoplasm",
  "term_id": "GO:0005737",
  "gene_symbol": "BTG1",
  "gene_name": "Protein BTG1"
}